gamma-aminobutyric acid catabolic process [GO:0009450] (biological process) Sources: GOC:ai Definition: The chemical reactions and pathways resulting in the breakdown of gamma-aminobutyric acid (GABA, 4-aminobutyrate), an amino acid which acts as a neurotransmitter in some organisms. Regulation: RO_0002211 by regulation of gamma-aminobutyric acid catabolic process [GO:1901715]; negatively regulated by GO:1901716; positively regulated by positive regulation of gamma-aminobutyric acid catabolic process [GO:1901717] Relationships: is_a amino acid catabolic process [GO:0009063]; is a type of gamma-aminobutyric acid metabolic process [GO:0009448]; is a type of non-proteinogenic amino acid catabolic process [GO:0170044] Also known as: 4-aminobutanoate catabolic process, 4-aminobutanoate catabolism, 4-aminobutyrate catabolic process, 4-aminobutyrate catabolism, GABA catabolic process, GABA catabolism, gamma-aminobutyric acid breakdown, gamma-aminobutyric acid catabolism, gamma-aminobutyric acid degradation Note: See also the biological process term 'neurotransmitter catabolic process ; GO:0042135'.